{
  "term_id": "GO:0005643",
  "gene": "UniProtKB:Q5VU65",
  "term_label": "nuclear pore",
  "gene_symbol": "NUP210L",
  "gene_name": "Nuclear pore membrane glycoprotein 210-like"
}